{
  "gene": "UniProtKB:Q5XLA6",
  "gene_name": "Putative caspase recruitment domain-containing protein 17P",
  "term_label": "Unknown biological process",
  "term_id": "UNKNOWN:0002",
  "gene_symbol": "CARD17P"
}